renal amino acid absorption [GO:1990297] (biological process) Definition: A renal system process in which amino acids are taken up from the collecting ducts, glomerulus and proximal and distal loops of the nephron. In non-mammalian species, absorption may occur in related structures. Relationships: is a type of renal absorption [GO:0070293] Regulation: regulated by GO:1902752; negatively regulated by negative regulation of renal amino acid absorption [GO:1902753]; positively regulated by positive regulation of renal amino acid absorption [GO:1902754] References: PMID:1526373 Sources: GOC:hjd